{
  "term_label": "neurotransmitter receptor transport, endosome to postsynaptic membrane",
  "gene_name": "Leucine-rich repeat-containing protein 7",
  "gene_symbol": "LRRC7",
  "gene": "UniProtKB:Q96NW7",
  "term_id": "GO:0098887"
}